{
  "gene": "UniProtKB:O15013",
  "term_id": "GO:0030036",
  "gene_symbol": "ARHGEF10",
  "gene_name": "Rho guanine nucleotide exchange factor 10",
  "term_label": "actin cytoskeleton organization"
}